{
  "term_id": "GO:0005737",
  "gene_symbol": "BOLL",
  "gene": "UniProtKB:Q8N9W6",
  "gene_name": "Protein boule-like",
  "term_label": "cytoplasm"
}